regulation of mesodermal cell differentiation [GO:1905770] (biological process) References: PMID:23765923 Sources: GOC:BHF, GOC:BHF_miRNA, GOC:TermGenie, GOC:rph, GO_REF:0000058 Definition: Any process that modulates the frequency, rate or extent of mesodermal cell differentiation. Subtypes: regulation of mesodermal cell fate specification [GO:0042661], GO:0048334, GO:1905771, positive regulation of mesodermal cell differentiation [GO:1905772] Relationships: is a type of regulation of cell differentiation [GO:0045595]; regulates GO:0048333 Also known as: regulation of mesoderm cell differentiation